{
  "gene_symbol": "TBX3",
  "gene_name": "T-box transcription factor TBX3",
  "gene": "UniProtKB:O15119",
  "term_label": "cell fate specification",
  "term_id": "GO:0001708"
}